{
  "gene_symbol": "C4A",
  "gene_name": "Complement C4-A",
  "gene": "UniProtKB:P0C0L4",
  "term_id": "UNKNOWN:0001",
  "term_label": "Unknown molecular function"
}